mitochondrial outer membrane translocase complex assembly [GO:0070096] (biological process) Sources: GOC:BHF, GOC:vk Also known as: TOM complex assembly, mitochondrion outer membrane translocase complex assembly Definition: The aggregation, arrangement and bonding together of a set of components to form a mitochondrial outer membrane translocase complex. Relationships: is a type of GO:0065003; is part of outer mitochondrial membrane organization [GO:0007008]